{
  "term_label": "sulfur compound metabolic process",
  "term_id": "GO:0006790",
  "gene_name": "Carbohydrate sulfotransferase 7",
  "gene_symbol": "CHST7",
  "gene": "UniProtKB:Q9NS84"
}